{
  "gene": "UniProtKB:P0DPH7",
  "term_id": "GO:0000278",
  "gene_symbol": "TUBA3C",
  "gene_name": "Tubulin alpha-3C chain",
  "term_label": "mitotic cell cycle"
}